{
  "gene_symbol": "CNN3",
  "term_label": "actin filament organization",
  "gene_name": "Calponin-3",
  "gene": "UniProtKB:Q15417",
  "term_id": "GO:0007015"
}